positive regulation of NK T cell differentiation [GO:0051138] (biological process) Definition: Any process that activates or increases the frequency, rate or extent of natural killer T cell differentiation. Note: Note that immunologists typically use the word 'development' to refer to cells of B or T cell lineages undergoing the process that GO describes as 'cell differentiation'. Also known as: positive regulation of NK T lymphocyte differentiation, positive regulation of NK T-cell differentiation, positive regulation of NK T-lymphocyte differentiation, positive regulation of NKT cell differentiation, positive regulation of NT cell differentiation, positive regulation of natural T cell differentiation, positive regulation of natural killer T cell differentiation, up regulation of NK T cell differentiation, up-regulation of NK T cell differentiation, upregulation of NK T cell differentiation, activation of NK T cell differentiation, stimulation of NK T cell differentiation, positive regulation of NK T cell development References: PMID:12154375, PMID:9133426 Sources: ISBN:0781735149 Relationships: is a type of positive regulation of alpha-beta T cell differentiation [GO:0046638]; is a type of regulation of NK T cell differentiation [GO:0051136]; RO_0002213 NK T cell differentiation [GO:0001865]